{
  "gene": "UniProtKB:Q86SZ2",
  "term_id": "UNKNOWN:0001",
  "gene_symbol": "TRAPPC6B",
  "gene_name": "Trafficking protein particle complex subunit 6B",
  "term_label": "Unknown molecular function"
}